{
  "term_label": "double-strand break repair via single-strand annealing",
  "gene": "UniProtKB:P43351",
  "term_id": "GO:0045002",
  "gene_symbol": "RAD52",
  "gene_name": "DNA repair protein RAD52 homolog"
}